{
  "gene": "UniProtKB:Q9P2P5",
  "term_label": "cytoplasm",
  "term_id": "GO:0005737",
  "gene_symbol": "HECW2",
  "gene_name": "E3 ubiquitin-protein ligase HECW2"
}